{
  "gene": "UniProtKB:Q15370",
  "term_id": "GO:0030891",
  "gene_name": "Elongin-B",
  "term_label": "VCB complex",
  "gene_symbol": "ELOB"
}